{
  "gene": "UniProtKB:A0A0C4DH38",
  "gene_symbol": "IGHV5-51",
  "term_id": "UNKNOWN:0003",
  "gene_name": "Immunoglobulin heavy variable 5-51",
  "term_label": "Unknown cellular component"
}